extrinsic component of cytoplasmic side of plasma membrane [GO:0031234] (cellular component) Note: Consider also annotating to 'cell cortex ; GO:0005938'. Also known as: extrinsic to internal leaflet of plasma membrane, extrinsic to internal side of plasma membrane, extrinsic to cytoplasmic side of plasma membrane Sources: GOC:mah Definition: The component of a plasma membrane consisting of gene products and protein complexes that are loosely bound to its cytoplasmic surface, but not integrated into the hydrophobic region. Relationships: is a type of extrinsic component of plasma membrane [GO:0019897]; is part of cytoplasmic side of plasma membrane [GO:0009898]